{
  "term_label": "olfactory receptor activity",
  "gene": "UniProtKB:Q96R69",
  "term_id": "GO:0004984",
  "gene_name": "Olfactory receptor 4F4",
  "gene_symbol": "OR4F4"
}